{
  "gene_symbol": "GRID2IP",
  "gene_name": "Delphilin",
  "term_label": "Unknown molecular function",
  "term_id": "UNKNOWN:0001",
  "gene": "UniProtKB:A4D2P6"
}